modulation of process of another organism [GO:0035821] (biological process) Definition: A process in which an organism effects a change in a biological process in another organism. Also known as: modification of morphology or physiology of other organism, modulation of process of other organism, regulation of morphology of other organism, regulation of physiological process of other organism, regulation of physiology of other organism, regulation of morphology or physiology of other organism Subtypes: venom-mediated perturbation of biological process [GO:0035738], symbiont-mediated perturbation of host process [GO:0044003], GO:0051709, GO:0051851, modulation of nutrient release by symbiont [GO:0052460] Relationships: is a type of biological process involved in interspecies interaction between organisms [GO:0044419] Sources: GOC:bf